{
  "term_id": "UNKNOWN:0001",
  "gene": "UniProtKB:Q8WU39",
  "gene_symbol": "MZB1",
  "gene_name": "Marginal zone B- and B1-cell-specific protein",
  "term_label": "Unknown molecular function"
}